{
  "term_id": "UNKNOWN:0003",
  "gene_name": "Olfactory receptor 5H6",
  "gene_symbol": "OR5H6",
  "gene": "UniProtKB:Q8NGV6",
  "term_label": "Unknown cellular component"
}